{
  "gene_name": "Double homeobox protein 4-like protein 7",
  "gene_symbol": "DUX4L7",
  "gene": "UniProtKB:P0CJ90",
  "term_id": "GO:0006357",
  "term_label": "regulation of transcription by RNA polymerase II"
}